{
  "gene_name": "Small ribosomal subunit protein uS3m",
  "gene_symbol": "MRPS24",
  "term_label": "Unknown biological process",
  "gene": "UniProtKB:Q96EL2",
  "term_id": "UNKNOWN:0002"
}